{
  "gene_name": "DNA replication licensing factor MCM5",
  "term_id": "GO:0003697",
  "term_label": "single-stranded DNA binding",
  "gene": "UniProtKB:P33992",
  "gene_symbol": "MCM5"
}